{
  "term_label": "Unknown cellular component",
  "gene": "UniProtKB:Q01167",
  "term_id": "UNKNOWN:0003",
  "gene_symbol": "FOXK2",
  "gene_name": "Forkhead box protein K2"
}